formin-nucleated actin cable organization [GO:0110009] (biological process) Definition: A process that results in the assembly, arrangement of constituent parts, or disassembly of a formin-nucleated actin cable. Relationships: is_a actin filament bundle organization [GO:0061572] Subtypes: GO:0070649 Sources: GOC:mah